compound eye retinal cell apoptotic process [GO:1990010] (biological process) References: PMID:12021768 Sources: GOC:mtg_apoptosis Definition: Any apoptotic process in a compound eye retinal cell. Relationships: is a type of GO:1990009 Regulation: regulated by regulation of compound eye retinal cell apoptotic process [GO:1901692]; negatively regulated by negative regulation of compound eye retinal cell apoptotic process [GO:1901693]; positively regulated by positive regulation of compound eye retinal cell apoptotic process [GO:1901694]